{
  "gene": "UniProtKB:P51114",
  "term_label": "translation regulator activity",
  "gene_symbol": "FXR1",
  "gene_name": "RNA-binding protein FXR1",
  "term_id": "GO:0045182"
}